{
  "gene_name": "Transforming growth factor-beta-induced protein ig-h3",
  "gene_symbol": "TGFBI",
  "term_label": "extracellular space",
  "term_id": "GO:0005615",
  "gene": "UniProtKB:Q15582"
}